anterior Malpighian tubule development [GO:0061327] (biological process) References: PMID:19783135 Sources: GOC:dph, GOC:mtg_kidney_jan10 Relationships: is a type of Malpighian tubule development [GO:0072002] Definition: The process whose specific outcome is the progression of the anterior Malpighian tubule over time, from its formation to the mature structure. The pair of anterior tubules arise from a dorsal region of the embryonic hindgut and projects forwards through the body cavity. A Malpighian tubule is a fine, thin-walled excretory tubule in insects which connects with the posterior part of the gut.